{
  "gene_name": "Late cornified envelope protein 2D",
  "term_label": "Unknown biological process",
  "term_id": "UNKNOWN:0002",
  "gene": "UniProtKB:Q5TA82",
  "gene_symbol": "LCE2D"
}